{
  "gene_symbol": "TVP23C",
  "gene": "UniProtKB:Q96ET8",
  "gene_name": "Golgi apparatus membrane protein TVP23 homolog C",
  "term_label": "vesicle-mediated transport",
  "term_id": "GO:0016192"
}